{
  "gene": "UniProtKB:Q76I76",
  "term_label": "actin binding",
  "gene_symbol": "SSH2",
  "gene_name": "Protein phosphatase Slingshot homolog 2",
  "term_id": "GO:0003779"
}